{
  "term_id": "UNKNOWN:0003",
  "gene": "UniProtKB:Q96FF7",
  "term_label": "Unknown cellular component",
  "gene_symbol": "MISP3",
  "gene_name": "Uncharacterized protein MISP3"
}